{
  "gene_symbol": "SCAF4",
  "term_id": "GO:2000805",
  "term_label": "negative regulation of termination of RNA polymerase II transcription, poly(A)-coupled",
  "gene": "UniProtKB:O95104",
  "gene_name": "SR-related and CTD-associated factor 4"
}